regulation of pentadecane biosynthetic process [GO:1900887] (biological process) Relationships: is a type of GO:1901577; RO_0002211 pentadecane biosynthetic process [GO:1900634] Definition: Any process that modulates the frequency, rate or extent of pentadecane biosynthetic process. Sources: GOC:TermGenie, GOC:mengo_curators Subtypes: negative regulation of pentadecane biosynthetic process [GO:1900888], GO:1900889 Also known as: regulation of pentadecane anabolism, regulation of pentadecane biosynthesis, regulation of pentadecane formation, regulation of pentadecane synthesis